{
  "gene_name": "Lethal(3)malignant brain tumor-like protein 2",
  "term_label": "negative regulation of DNA-templated transcription",
  "gene_symbol": "L3MBTL2",
  "term_id": "GO:0045892",
  "gene": "UniProtKB:Q969R5"
}